positive regulation of organic acid transport [GO:0032892] (biological process) Relationships: is a type of regulation of organic acid transport [GO:0032890]; is a type of positive regulation of transport [GO:0051050]; positively regulates organic acid transport [GO:0015849] Definition: Any process that activates or increases the frequency, rate or extent of the directed movement of organic acids into, out of or within a cell, or between cells, by means of some agent such as a transporter or pore. Sources: GOC:mah Also known as: up regulation of organic acid transport, up-regulation of organic acid transport, upregulation of organic acid transport, activation of organic acid transport, stimulation of organic acid transport Subtypes: positive regulation of L-glutamate import across plasma membrane [GO:0002038], GO:0014049, positive regulation of gamma-aminobutyric acid secretion [GO:0014054], GO:0035432, positive regulation of gamma-aminobutyric acid uptake involved in transmission of nerve impulse [GO:0051950], positive regulation of bile acid secretion [GO:0120189], positive regulation of D-aspartate import across plasma membrane [GO:0140217], GO:1900925, positive regulation of L-threonine import across plasma membrane [GO:1900928], GO:1900931, positive regulation of proline import across plasma membrane [GO:1902836], positive regulation of aspartate secretion [GO:1904450], positive regulation of glycine secretion, neurotransmission [GO:1904626], positive regulation of L-lysine import across plasma membrane [GO:1905010], positive regulation of L-leucine import across plasma membrane [GO:1905534], positive regulation of L-arginine import across plasma membrane [GO:1905589], positive regulation of L-methionine import across plasma membrane [GO:1905626], positive regulation of fatty acid transport [GO:2000193], positive regulation of glutamine transport [GO:2000487]